{
  "gene_symbol": "SPRY4",
  "gene": "UniProtKB:Q9C004",
  "term_label": "Unknown cellular component",
  "term_id": "UNKNOWN:0003",
  "gene_name": "Protein sprouty homolog 4"
}